{
  "term_label": "blood vessel development",
  "gene_name": "Teratocarcinoma-derived growth factor 1",
  "gene_symbol": "TDGF1",
  "gene": "UniProtKB:P13385",
  "term_id": "GO:0001568"
}